{
  "gene": "UniProtKB:P11047",
  "gene_symbol": "LAMC1",
  "gene_name": "Laminin subunit gamma-1",
  "term_id": "GO:0005615",
  "term_label": "extracellular space"
}